{
  "term_id": "GO:0005634",
  "gene_symbol": "UBC",
  "term_label": "nucleus",
  "gene": "UniProtKB:P0CG48",
  "gene_name": "Polyubiquitin-C"
}